{
  "gene_name": "Serine_threonine-protein phosphatase 4 regulatory subunit 2",
  "term_label": "protein phosphatase regulator activity",
  "gene_symbol": "PPP4R2",
  "term_id": "GO:0019888",
  "gene": "UniProtKB:Q9NY27"
}